hydrogen peroxide biosynthetic process [GO:0050665] (biological process) Sources: GOC:ai Also known as: H2O2 biosynthetic process, hydrogen peroxide anabolism, hydrogen peroxide biosynthesis, hydrogen peroxide formation, hydrogen peroxide generation, hydrogen peroxide synthesis Definition: The chemical reactions and pathways resulting in the formation of hydrogen peroxide (H2O2), a potentially harmful byproduct of aerobic cellular respiration which can cause damage to DNA. Relationships: is a type of GO:0042743; is a type of reactive oxygen species biosynthetic process [GO:1903409] Regulation: regulated by GO:0010728; positively regulated by positive regulation of hydrogen peroxide biosynthetic process [GO:0010729]; negatively regulated by GO:0010730